{
  "gene_name": "Cyclin-dependent kinase inhibitor 1",
  "gene": "UniProtKB:P38936",
  "term_id": "GO:0000307",
  "gene_symbol": "CDKN1A",
  "term_label": "cyclin-dependent protein kinase holoenzyme complex"
}